{
  "term_label": "positive regulation of transcription by RNA polymerase II",
  "gene_symbol": "RXRB",
  "gene": "UniProtKB:P28702",
  "term_id": "GO:0045944",
  "gene_name": "Retinoic acid receptor RXR-beta"
}